{
  "gene_name": "Monocarboxylate transporter 7",
  "gene_symbol": "SLC16A6",
  "term_label": "monocarboxylic acid transmembrane transporter activity",
  "term_id": "GO:0008028",
  "gene": "UniProtKB:O15403"
}